{
  "term_label": "transforming growth factor beta receptor signaling pathway",
  "gene_symbol": "ITGB5",
  "term_id": "GO:0007179",
  "gene_name": "Integrin beta-5",
  "gene": "UniProtKB:P18084"
}